{
  "term_id": "GO:0005886",
  "gene_name": "Rho GTPase-activating protein 9",
  "gene_symbol": "ARHGAP9",
  "term_label": "plasma membrane",
  "gene": "UniProtKB:Q9BRR9"
}